{
  "gene_name": "Leukotriene A-4 hydrolase",
  "term_label": "leukotriene biosynthetic process",
  "gene_symbol": "LTA4H",
  "term_id": "GO:0019370",
  "gene": "UniProtKB:P09960"
}